{
  "gene_symbol": "BACH1",
  "gene_name": "Transcription regulator protein BACH1",
  "term_id": "GO:0006357",
  "gene": "UniProtKB:O14867",
  "term_label": "regulation of transcription by RNA polymerase II"
}